{
  "gene": "UniProtKB:Q9H553",
  "gene_symbol": "ALG2",
  "term_id": "GO:0012505",
  "gene_name": "Alpha-1,3_1,6-mannosyltransferase ALG2",
  "term_label": "endomembrane system"
}